{
  "term_label": "regulation of protein stability",
  "gene": "UniProtKB:Q93008",
  "gene_name": "Probable ubiquitin carboxyl-terminal hydrolase FAF-X",
  "gene_symbol": "USP9X",
  "term_id": "GO:0031647"
}